{
  "gene_symbol": "REEP1",
  "gene": "UniProtKB:Q9H902",
  "gene_name": "Receptor expression-enhancing protein 1",
  "term_label": "olfactory receptor binding",
  "term_id": "GO:0031849"
}